{
  "gene": "UniProtKB:Q13637",
  "gene_symbol": "RAB32",
  "gene_name": "Ras-related protein Rab-32",
  "term_id": "GO:0005802",
  "term_label": "trans-Golgi network"
}